{
  "gene_name": "Tetratricopeptide repeat protein 31",
  "term_label": "Unknown biological process",
  "gene_symbol": "TTC31",
  "gene": "UniProtKB:Q49AM3",
  "term_id": "UNKNOWN:0002"
}